regulation of astrocyte activation [GO:0061888] (BP) Definition: Any process that modulates the frequency, rate or extent of astrocyte activation. References: PMID:20005821 Sources: GOC:aruk, GOC:bc Subtypes: negative regulation of astrocyte activation [GO:0061889], GO:0061890 Relationships: is a type of GO:0048710; is a type of GO:0050865; regulates GO:0048143